{
  "term_label": "membrane",
  "gene_symbol": "NBEA",
  "gene": "UniProtKB:Q8NFP9",
  "gene_name": "Neurobeachin",
  "term_id": "GO:0016020"
}